ribose phosphate diphosphokinase activity [GO:0004749] (molecular function) Note: Note that this term has a MetaCyc pathway reference as the pathway only has a single step. Also known as: ribose-phosphate pyrophosphokinase activity, 5-phosphoribose pyrophosphorylase activity, 5-phosphoribosyl-1-pyrophosphate synthetase activity, 5-phosphoribosyl-alpha-1-pyrophosphate synthetase activity, ATP:D-ribose-5-phosphate diphosphotransferase activity, PP-ribose P synthetase activity, PPRibP synthetase activity, PRPP synthetase activity, phosphoribosyl diphosphate synthetase activity, phosphoribosyl pyrophosphate synthetase activity, phosphoribosyl-diphosphate synthetase activity, phosphoribosylpyrophosphate synthase activity, phosphoribosylpyrophosphate synthetase activity, pyrophosphoribosylphosphate synthetase activity, ribophosphate pyrophosphokinase activity, ribose-5-phosphate pyrophosphokinase activity, ribose-phosphate diphosphokinase activity Relationships: is a type of diphosphotransferase activity [GO:0016778] Sources: RHEA:15609 Definition: Catalysis of the reaction: D-ribose 5-phosphate + ATP = 5-phospho-alpha-D-ribose 1-diphosphate + AMP + 2 H+.